{
  "gene_symbol": "MGAM",
  "gene_name": "Maltase-glucoamylase",
  "term_id": "GO:0004558",
  "term_label": "alpha-1,4-glucosidase activity",
  "gene": "UniProtKB:O43451"
}